{
  "gene": "UniProtKB:P43631",
  "gene_name": "Killer cell immunoglobulin-like receptor 2DS2",
  "gene_symbol": "KIR2DS2",
  "term_label": "immune receptor activity",
  "term_id": "GO:0140375"
}